{
  "gene": "UniProtKB:O75473",
  "term_id": "GO:0005886",
  "gene_symbol": "LGR5",
  "term_label": "plasma membrane",
  "gene_name": "Leucine-rich repeat-containing G-protein coupled receptor 5"
}